{
  "term_id": "UNKNOWN:0002",
  "gene": "UniProtKB:A0A8Q3SIZ7",
  "gene_name": "Uncharacterized protein",
  "term_label": "Unknown biological process",
  "gene_symbol": "A0A8Q3SIZ7"
}